cell proliferation in hindbrain ventricular zone [GO:0021923] (biological process) Definition: The multiplication or reproduction of cells, resulting in the expansion of a cell population in the hindbrain region that is adjacent to the ventricular cavity. Subtypes: cerebellar Purkinje cell precursor proliferation [GO:0021925], Golgi cell precursor proliferation [GO:0021926], deep nuclear neuron precursor proliferation [GO:0021927], GO:0021928, GO:0021929 Relationships: is a type of GO:0021534 References: PMID:12593981, PMID:15157725 Sources: GOC:cls, GOC:dgh, GOC:dph, GOC:jid, GO_REF:0000021